{
  "gene": "UniProtKB:P48681",
  "gene_name": "Nestin",
  "gene_symbol": "NES",
  "term_label": "positive regulation of intermediate filament depolymerization",
  "term_id": "GO:0030844"
}